mannokinase activity [GO:0019158] (molecular function) Definition: Catalysis of the reaction: ATP + D-mannose = ADP + D-mannose 6-phosphate. Relationships: is a type of GO:0004396 Sources: EC:2.7.1.7 Also known as: ATP:D-mannose 6-phosphotransferase activity, D-fructose (D-mannose) kinase activity, mannokinase (phosphorylating)